{
  "gene": "UniProtKB:Q6PF18",
  "gene_symbol": "MORN3",
  "term_label": "Unknown molecular function",
  "gene_name": "MORN repeat-containing protein 3",
  "term_id": "UNKNOWN:0001"
}